{
  "gene": "UniProtKB:Q13322",
  "gene_name": "Growth factor receptor-bound protein 10",
  "term_label": "intracellular signal transduction",
  "gene_symbol": "GRB10",
  "term_id": "GO:0035556"
}